{
  "gene": "UniProtKB:Q8WXE1",
  "gene_symbol": "ATRIP",
  "term_id": "UNKNOWN:0001",
  "term_label": "Unknown molecular function",
  "gene_name": "ATR-interacting protein"
}